DNA restriction-modification system [GO:0009307] (BP) Also known as: DNA restriction Definition: A defense process found in many bacteria and archaea that protects the organism from invading foreign DNA by cleaving it with a restriction endonuclease. The organism's own DNA is protected by methylation of a specific nucleotide, which occurs immediately following replication, in the same target site as the restriction enzyme. Relationships: is a type of GO:0006304; is a type of GO:0044355 Sources: GOC:jl, UniProtKB-KW:KW-0680